{
  "gene": "UniProtKB:Q6N022",
  "term_label": "protein homodimerization activity",
  "gene_name": "Teneurin-4",
  "gene_symbol": "TENM4",
  "term_id": "GO:0042803"
}